regulation of aggregation involved in sorocarp development [GO:0060176] (biological process) Sources: GOC:dph, GOC:tb Definition: Any process that modulates the frequency, rate or extent of aggregation during sorocarp development. Aggregation involved in sorocarp development is the process whose specific outcome is the progression of the aggregate over time, from its formation to the point when a slug is formed. Aggregate development begins in response to starvation and continues by the chemoattractant-mediated movement of cells toward each other. The aggregate is a multicellular structure that gives rise to the slug. Subtypes: regulation of aggregate size involved in sorocarp development [GO:0031157], GO:0110013, negative regulation of aggregation involved in sorocarp development [GO:0110014] Relationships: is a type of regulation of response to nutrient levels [GO:0032107]; is a type of regulation of developmental process [GO:0050793]; is a type of regulation of cellular response to stress [GO:0080135]; regulates aggregation involved in sorocarp development [GO:0031152]